{
  "term_label": "Z disc",
  "gene_symbol": "CASQ2",
  "gene": "UniProtKB:O14958",
  "term_id": "GO:0030018",
  "gene_name": "Calsequestrin-2"
}